{
  "term_id": "UNKNOWN:0002",
  "gene_name": "Uncharacterized protein encoded by LINC02876",
  "term_label": "Unknown biological process",
  "gene_symbol": "LINC02876",
  "gene": "UniProtKB:F2Z3M2"
}